{
  "term_label": "intracellular signal transduction",
  "gene_name": "Ras-associated and pleckstrin homology domains-containing protein 1",
  "term_id": "GO:0035556",
  "gene_symbol": "RAPH1",
  "gene": "UniProtKB:Q70E73"
}